prothoracic disc morphogenesis [GO:0007470] (biological process) Definition: The process in which the anatomical structures derived from the prothoracic disc are generated and organized. This includes the transformation of a prothoracic imaginal disc from a monolayered epithelium in the larvae of holometabolous insects into the recognizable adult humerous and anterior spiracle. Sources: GOC:bf, ISBN:0879694238 Also known as: prothoracic disc metamorphosis Relationships: is a type of imaginal disc morphogenesis [GO:0007560]; is part of prothoracic disc development [GO:0035219]